{
  "gene": "UniProtKB:Q9ULG1",
  "gene_name": "Chromatin-remodeling ATPase INO80",
  "term_id": "GO:0006281",
  "term_label": "DNA repair",
  "gene_symbol": "INO80"
}